{
  "term_id": "GO:0006357",
  "gene_name": "Lysine-specific demethylase 3A",
  "term_label": "regulation of transcription by RNA polymerase II",
  "gene": "UniProtKB:Q9Y4C1",
  "gene_symbol": "KDM3A"
}